{
  "gene_symbol": "LYST",
  "gene_name": "Lysosomal-trafficking regulator",
  "term_id": "GO:0007040",
  "gene": "UniProtKB:Q99698",
  "term_label": "lysosome organization"
}